{
  "gene": "UniProtKB:Q7Z2K8",
  "term_id": "GO:0005886",
  "gene_name": "G protein-regulated inducer of neurite outgrowth 1",
  "term_label": "plasma membrane",
  "gene_symbol": "GPRIN1"
}